{
  "gene_name": "Glycogenin-2",
  "gene": "UniProtKB:O15488",
  "term_label": "cytoplasm",
  "term_id": "GO:0005737",
  "gene_symbol": "GYG2"
}